{
  "gene_name": "Immunoglobulin lambda variable 3-27",
  "gene_symbol": "IGLV3-27",
  "gene": "UniProtKB:P01718",
  "term_label": "immunoglobulin complex",
  "term_id": "GO:0019814"
}